{
  "gene": "UniProtKB:Q13469",
  "term_label": "RNA polymerase II cis-regulatory region sequence-specific DNA binding",
  "gene_symbol": "NFATC2",
  "term_id": "GO:0000978",
  "gene_name": "Nuclear factor of activated T-cells, cytoplasmic 2"
}